{
  "gene_name": "WD40 repeat-containing protein SMU1",
  "term_id": "GO:0071011",
  "gene_symbol": "SMU1",
  "term_label": "precatalytic spliceosome",
  "gene": "UniProtKB:Q2TAY7"
}